tRNA destabilization [GO:0036417] (biological process) Relationships: is a type of regulation of tRNA stability [GO:0036415]; is a type of RNA destabilization [GO:0050779]; is a type of GO:1902372 Sources: GOC:aa, GOC:bf Definition: Any process that decreases the stability of a tRNA molecule, making it more vulnerable to degradative processes.